fatty acid methyl ester metabolic process [GO:1902898] (biological process) Also known as: FAME metabolic process, fatty acid methyl ester metabolism Subtypes: GO:1902899 Relationships: is a type of fatty acid derivative metabolic process [GO:1901568] Definition: The chemical reactions and pathways involving fatty acid methyl ester. References: PMID:16570218 Sources: GOC:TermGenie, GOC:mengo_curators, GO_REF:0000068